{
  "gene": "UniProtKB:O75534",
  "gene_name": "Cold shock domain-containing protein E1",
  "term_label": "mCRD-mediated mRNA stability complex",
  "term_id": "GO:0106002",
  "gene_symbol": "CSDE1"
}